{
  "gene": "UniProtKB:Q13439",
  "gene_symbol": "GOLGA4",
  "gene_name": "Golgin subfamily A member 4",
  "term_id": "GO:0005794",
  "term_label": "Golgi apparatus"
}